{
  "term_id": "GO:0002227",
  "gene_symbol": "H2BC12",
  "term_label": "innate immune response in mucosa",
  "gene": "UniProtKB:O60814",
  "gene_name": "Histone H2B type 1-K"
}